{
  "term_id": "GO:0000981",
  "gene": "UniProtKB:Q15306",
  "gene_name": "Interferon regulatory factor 4",
  "term_label": "DNA-binding transcription factor activity, RNA polymerase II-specific",
  "gene_symbol": "IRF4"
}